{
  "gene_symbol": "BZW1",
  "gene": "UniProtKB:Q7L1Q6",
  "term_label": "Unknown molecular function",
  "gene_name": "eIF5-mimic protein 2",
  "term_id": "UNKNOWN:0001"
}